{
  "term_label": "nucleus",
  "gene": "UniProtKB:Q14106",
  "gene_symbol": "TOB2",
  "gene_name": "Protein Tob2",
  "term_id": "GO:0005634"
}